dolipore septum [GO:0000937] (cellular component) Sources: GOC:clt Definition: A septum, or cross-wall, between two portions of a cell or hypha; contains a central pore around which the septum is swollen to form a barrel-shaped structure; pore is covered on each side of the septum by a septal pore cap (parenthosome). Relationships: is a type of porous cell septum [GO:0000934]